negative regulation of endothelial cell-matrix adhesion [GO:1904905] (biological process) Definition: Any process that stops, prevents or reduces the frequency, rate or extent of endothelial cell-matrix adhesion. References: PMID:19460962 Sources: GOC:BHF, GOC:BHF_miRNA, GOC:TermGenie, GOC:bc, GO_REF:0000058 Also known as: down regulation of endothelial cell-matrix adhesion, down-regulation of endothelial cell-matrix adhesion, downregulation of endothelial cell-matrix adhesion, inhibition of endothelial cell-matrix adhesion Relationships: is a type of negative regulation of cell-matrix adhesion [GO:0001953]; is a type of regulation of endothelial cell-matrix adhesion [GO:1904904]; negatively regulates endothelial cell-matrix adhesion [GO:0090673]